{
  "gene": "UniProtKB:Q9NWZ3",
  "gene_symbol": "IRAK4",
  "term_id": "GO:0019221",
  "term_label": "cytokine-mediated signaling pathway",
  "gene_name": "Interleukin-1 receptor-associated kinase 4"
}